{
  "gene": "UniProtKB:Q9UM22",
  "gene_symbol": "EPDR1",
  "term_label": "Unknown molecular function",
  "gene_name": "Mammalian ependymin-related protein 1",
  "term_id": "UNKNOWN:0001"
}